(13E)-labda-7,13-dien-15-ol synthase activity [GO:0102305] (molecular function) Definition: Catalysis of the reaction: geranylgeranyl diphosphate + H2O = (13E)-labda-7,13-dien-15-ol + diphosphate. Sources: RHEA:32075 Relationships: is a type of GO:0016794